negative regulation of protein localization to cell periphery [GO:1904376] (biological process) Subtypes: negative regulation of protein localization to plasma membrane [GO:1903077], negative regulation of protein localization to ciliary membrane [GO:1903568], negative regulation of protein localization to basolateral plasma membrane [GO:1904509], negative regulation of protein localization to cell cortex [GO:1904777] Also known as: down regulation of protein localization to cell periphery, down-regulation of protein localization to cell periphery, downregulation of protein localization to cell periphery, inhibition of protein localization to cell periphery Definition: Any process that stops, prevents or reduces the frequency, rate or extent of protein localization to cell periphery. Relationships: is a type of negative regulation of protein localization [GO:1903828]; is a type of regulation of protein localization to cell periphery [GO:1904375]; negatively regulates protein localization to cell periphery [GO:1990778] References: PMID:18216290 Sources: GOC:TermGenie, GO_REF:0000058